N-acetylneuraminate catabolic process [GO:0019262] (biological process) Relationships: is a type of GO:0006054; is a type of amino sugar catabolic process [GO:0046348]; is a type of carboxylic acid catabolic process [GO:0046395] Sources: ISBN:0198506732 Also known as: N-acetylneuraminate breakdown, N-acetylneuraminate catabolism, N-acetylneuraminate degradation Definition: The chemical reactions and pathways resulting in the breakdown of N-acetylneuraminate, the anion of 5-(acetylamino)-3,5-dideoxy-D-glycero-D-galacto-non-3-ulosonic acid.